p-benzoquinone reductase (NADPH) activity [GO:0018541] (molecular function) Definition: Catalysis of the reaction: 1,4-benzoquinone + H+ + NADPH = hydroquinone + NADP+. Also known as: NADPH:p-benzoquinone oxidoreductase activity Sources: RHEA:23488 Relationships: is a type of oxidoreductase activity, acting on NAD(P)H, quinone or similar compound as acceptor [GO:0016655]